{
  "gene_symbol": "TBC1D23",
  "gene": "UniProtKB:Q9NUY8",
  "gene_name": "TBC1 domain family member 23",
  "term_id": "UNKNOWN:0001",
  "term_label": "Unknown molecular function"
}